{
  "term_id": "GO:0031629",
  "gene_name": "Syntaxin-2",
  "term_label": "synaptic vesicle fusion to presynaptic active zone membrane",
  "gene": "UniProtKB:P32856",
  "gene_symbol": "STX2"
}